{
  "gene": "UniProtKB:P22732",
  "gene_name": "Solute carrier family 2, facilitated glucose transporter member 5",
  "term_label": "plasma membrane",
  "gene_symbol": "SLC2A5",
  "term_id": "GO:0005886"
}